{
  "term_label": "GTPase activity",
  "gene_name": "Ras-related protein Rab-13",
  "term_id": "GO:0003924",
  "gene_symbol": "RAB13",
  "gene": "UniProtKB:P51153"
}